negative regulation of fatty acid oxidation [GO:0046322] (biological process) Sources: GOC:ai Relationships: is a type of negative regulation of fatty acid metabolic process [GO:0045922]; is a type of regulation of fatty acid oxidation [GO:0046320]; negatively regulates GO:0019395 Definition: Any process that stops, prevents, or reduces the frequency, rate or extent of fatty acid oxidation. Subtypes: GO:0031999 Also known as: down regulation of fatty acid oxidation, down-regulation of fatty acid oxidation, downregulation of fatty acid oxidation, inhibition of fatty acid oxidation